{
  "gene_name": "Annexin A13",
  "term_label": "nucleus",
  "term_id": "GO:0005634",
  "gene_symbol": "ANXA13",
  "gene": "UniProtKB:P27216"
}